positive regulation of G1/S transition of mitotic cell cycle [GO:1900087] (biological process) Subtypes: traversing start control point of mitotic cell cycle [GO:0007089] Definition: Any signaling pathway that increases or activates a cell cycle cyclin-dependent protein kinase to modulate the switch from G1 phase to S phase of the mitotic cell cycle. Sources: GOC:mtg_cell_cycle Relationships: is_a positive regulation of mitotic cell cycle phase transition [GO:1901992]; is a type of positive regulation of cell cycle G1/S phase transition [GO:1902808]; is a type of regulation of G1/S transition of mitotic cell cycle [GO:2000045]; positively regulates G1/S transition of mitotic cell cycle [GO:0000082] Also known as: up regulation of G1/S transition of mitotic cell cycle, up-regulation of G1/S transition of mitotic cell cycle, upregulation of G1/S transition of mitotic cell cycle, activation of G1/S transition of mitotic cell cycle